{
  "gene_name": "Endothelial PAS domain-containing protein 1",
  "term_id": "GO:0005667",
  "gene": "UniProtKB:Q99814",
  "term_label": "transcription regulator complex",
  "gene_symbol": "EPAS1"
}